{
  "term_id": "UNKNOWN:0002",
  "gene_symbol": "WDR88",
  "gene": "UniProtKB:Q6ZMY6",
  "gene_name": "WD repeat-containing protein 88",
  "term_label": "Unknown biological process"
}